{
  "term_label": "zinc ion transmembrane transporter activity",
  "term_id": "GO:0005385",
  "gene_name": "Zinc transporter ZIP11",
  "gene_symbol": "SLC39A11",
  "gene": "UniProtKB:Q8N1S5"
}